{
  "term_id": "GO:0003712",
  "gene_name": "Probable JmjC domain-containing histone demethylation protein 2C",
  "gene_symbol": "JMJD1C",
  "gene": "UniProtKB:Q15652",
  "term_label": "transcription coregulator activity"
}